amino acid transport [GO:0006865] (biological process) Relationships: is a type of GO:0006810 Sources: GOC:ai Subtypes: amino acid transmembrane transport [GO:0003333], extracellular amino acid transport [GO:0006860], acidic amino acid transport [GO:0015800], GO:0015802, neutral amino acid transport [GO:0015804], L-amino acid transport [GO:0015807], gamma-aminobutyric acid transport [GO:0015812], methionine transport [GO:0015821], ornithine transport [GO:0015822], tryptophan transport [GO:0015827], hydroxyproline transport [GO:0034589], D-amino acid transport [GO:0042940], GO:0043090, GO:0051933 Definition: The directed movement of amino acids, organic acids containing one or more amino substituents, into, out of or within a cell, or between cells, by means of some agent such as a transporter or pore. Regulation: RO_0002211 by GO:0051955; negatively regulated by GO:0051956; positively regulated by positive regulation of amino acid transport [GO:0051957]